{
  "gene_symbol": "HSPA14",
  "gene": "UniProtKB:Q0VDF9",
  "term_label": "cytoplasm",
  "term_id": "GO:0005737",
  "gene_name": "Heat shock 70 kDa protein 14"
}